{
  "gene": "UniProtKB:P42574",
  "gene_symbol": "CASP3",
  "gene_name": "Caspase-3",
  "term_id": "GO:0008047",
  "term_label": "enzyme activator activity"
}